fat cell apoptotic process [GO:1904606] (biological process) Regulation: regulated by regulation of fat cell apoptotic process [GO:1904649]; negatively regulated by negative regulation of fat cell apoptotic process [GO:1904650]; positively regulated by GO:1904651 Also known as: adipocyte apoptotic process, adipose cell apoptotic process, adipocyte apoptosis, adipose cell apoptosis, fat cell apoptosis References: PMID:17024416 Sources: GOC:TermGenie, GO_REF:0000085 Relationships: is a type of apoptotic process [GO:0006915] Definition: Any apoptotic process in a fat cell.